{
  "term_id": "GO:0031982",
  "gene": "UniProtKB:Q96M98",
  "gene_name": "Parkin coregulated gene protein",
  "term_label": "vesicle",
  "gene_symbol": "PACRG"
}